{
  "gene_symbol": "KLHL8",
  "term_id": "GO:0031463",
  "gene_name": "Kelch-like protein 8",
  "term_label": "Cul3-RING ubiquitin ligase complex",
  "gene": "UniProtKB:Q9P2G9"
}